{
  "gene": "UniProtKB:Q9H7J1",
  "gene_symbol": "PPP1R3E",
  "gene_name": "Protein phosphatase 1 regulatory subunit 3E",
  "term_id": "GO:2001069",
  "term_label": "glycogen binding"
}